{
  "term_label": "calcium ion sensor activity",
  "term_id": "GO:0061891",
  "gene_name": "EF-hand domain-containing protein D1",
  "gene_symbol": "EFHD1",
  "gene": "UniProtKB:Q9BUP0"
}